TOM complex [GO:0140596] (cellular component) Definition: A large mitochondrial outer membrane translocase complex that mediates transport of proteins into mitochondrial compartments. TOM transports beta-barrel precursors across the outer membrane and the sorting and assembly machinery (SAM complex) inserts them into the target membrane. References: PMID:33035511 Also known as: translocase of the outer mitochondrial membrane Relationships: is a type of mitochondrial outer membrane translocase complex [GO:0005742]